{
  "gene_symbol": "SH3BGR",
  "gene_name": "SH3 domain-binding glutamic acid-rich protein",
  "gene": "UniProtKB:P55822",
  "term_id": "UNKNOWN:0002",
  "term_label": "Unknown biological process"
}